{
  "term_id": "GO:0007186",
  "gene_name": "Mas-related G-protein coupled receptor member G",
  "gene": "UniProtKB:Q86SM5",
  "gene_symbol": "MRGPRG",
  "term_label": "G protein-coupled receptor signaling pathway"
}